gamma-delta intraepithelial T cell differentiation [GO:0002304] (biological process) Relationships: is a type of gamma-delta T cell differentiation [GO:0042492] Also known as: gamma-delta intraepithelial T lymphocyte differentiation, gamma-delta intraepithelial T-cell differentiation, gamma-delta intraepithelial T-lymphocyte differentiation, gamma-delta intraepithelial T cell development Definition: The process in which a precursor cell type acquires the specialized features of a gamma-delta intraepithelial T cell. Intraepithelial T cells are found among epithelial cells in mucosal areas and have distinct phenotypes and developmental pathways. Note: Note that immunologists typically use the word 'development' to refer to cells of B or T cell lineages undergoing the process that GO describes as 'cell differentiation'. Subtypes: CD8-positive, gamma-delta intraepithelial T cell differentiation [GO:0002305], CD4-positive gamma-delta intraepithelial T cell differentiation [GO:0002306] Sources: GOC:add, ISBN:0781735149